{
  "term_id": "GO:0005634",
  "gene_symbol": "FUS",
  "term_label": "nucleus",
  "gene_name": "RNA-binding protein FUS",
  "gene": "UniProtKB:P35637"
}